di-trans, poly-cis-undecaprenol kinase activity [GO:0036433] (molecular function) Relationships: is a type of GO:0009038 Also known as: ditrans,polycis-undecaprenol kinase activity Definition: Catalysis of the reaction: di-trans, octa-cis-undecaprenol + ATP = di-trans,octa-cis-undecaprenyl phosphate + ADP + H+. Sources: RHEA:28122